esterosome lumen [GO:0034467] (cellular component) Relationships: is a type of cytoplasmic vesicle lumen [GO:0060205]; is part of GO:0033117 Sources: GOC:rph Definition: The volume enclosed by the membrane of an esterosome.